{
  "gene": "UniProtKB:Q75QN2",
  "term_id": "GO:0034472",
  "term_label": "snRNA 3'-end processing",
  "gene_name": "Integrator complex subunit 8",
  "gene_symbol": "INTS8"
}